methylmalonyl-CoA epimerase activity [GO:0004493] (molecular function) Relationships: is a type of racemase and epimerase activity [GO:0016854] Also known as: 2-methyl-3-oxopropanoyl-CoA 2-epimerase activity, DL-methylmalonyl-CoA racemase activity, methylmalonyl coenzyme A racemase activity, methylmalonyl-CoA 2-epimerase activity, methylmalonyl-CoA racemase activity Sources: EC:5.1.99.1, RHEA:20553 Definition: Catalysis of the reaction: (R)-methylmalonyl-CoA = (S)-methylmalonyl-CoA.